{
  "gene": "UniProtKB:Q9Y2Q9",
  "gene_name": "Small ribosomal subunit protein bS1m",
  "term_id": "UNKNOWN:0002",
  "gene_symbol": "MRPS28",
  "term_label": "Unknown biological process"
}